{
  "term_id": "GO:0043161",
  "gene_symbol": "KLHL2",
  "gene": "UniProtKB:O95198",
  "term_label": "proteasome-mediated ubiquitin-dependent protein catabolic process",
  "gene_name": "Kelch-like protein 2"
}